{
  "term_id": "GO:0030550",
  "gene": "UniProtKB:P0DTL4",
  "gene_symbol": "LY6S",
  "gene_name": "Lymphocyte antigen 6S",
  "term_label": "acetylcholine receptor inhibitor activity"
}